{
  "gene_name": "Uncharacterized protein C8orf88",
  "term_id": "GO:0030371",
  "gene": "UniProtKB:P0DMB2",
  "gene_symbol": "C8orf88",
  "term_label": "translation repressor activity"
}